{
  "gene_name": "Potassium_sodium hyperpolarization-activated cyclic nucleotide-gated channel 3",
  "term_id": "GO:0030425",
  "gene_symbol": "HCN3",
  "term_label": "dendrite",
  "gene": "UniProtKB:Q9P1Z3"
}